{
  "gene_name": "CD160 antigen",
  "term_label": "Unknown biological process",
  "gene_symbol": "CD160",
  "term_id": "UNKNOWN:0002",
  "gene": "UniProtKB:O95971"
}